{
  "term_label": "Unknown molecular function",
  "gene": "UniProtKB:Q9BYN8",
  "gene_symbol": "MRPS26",
  "gene_name": "Small ribosomal subunit protein mS26",
  "term_id": "UNKNOWN:0001"
}